{
  "term_label": "ciliary basal body",
  "term_id": "GO:0036064",
  "gene_symbol": "NPHP4",
  "gene": "UniProtKB:O75161",
  "gene_name": "Nephrocystin-4"
}